{
  "gene_symbol": "WDR59",
  "gene": "UniProtKB:Q6PJI9",
  "gene_name": "GATOR complex protein WDR59",
  "term_id": "GO:0035591",
  "term_label": "signaling adaptor activity"
}